{
  "gene_name": "Copine-7",
  "gene_symbol": "CPNE7",
  "term_label": "plasma membrane",
  "term_id": "GO:0005886",
  "gene": "UniProtKB:Q9UBL6"
}